pollen aperture [GO:0062074] (cellular component) Definition: An area where exine is reduced or absent, in the pollen wall. Relationships: is a type of cellular anatomical structure [GO:0110165]; is part of pollen wall [GO:0043667] References: PMID:30150313